{
  "gene": "UniProtKB:Q8IX94",
  "gene_symbol": "CTAGE4",
  "gene_name": "cTAGE family member 4",
  "term_label": "endoplasmic reticulum to Golgi vesicle-mediated transport",
  "term_id": "GO:0006888"
}